{
  "term_label": "Unknown biological process",
  "term_id": "UNKNOWN:0002",
  "gene": "UniProtKB:Q5VT28",
  "gene_symbol": "FAM27C",
  "gene_name": "Protein FAM27A_B_C"
}